{
  "term_label": "Unknown molecular function",
  "gene_symbol": "GOLGA2",
  "term_id": "UNKNOWN:0001",
  "gene_name": "Golgin subfamily A member 2",
  "gene": "UniProtKB:Q08379"
}